antigen processing and presentation of peptide antigen [GO:0048002] (biological process) Definition: The process in which an antigen-presenting cell expresses peptide antigen in association with an MHC protein complex on its cell surface, including proteolysis and transport steps for the peptide antigen both prior to and following assembly with the MHC protein complex. The peptide antigen is typically, but not always, processed from an endogenous or exogenous protein. Regulation: regulated by regulation of antigen processing and presentation of peptide antigen [GO:0002583]; negatively regulated by negative regulation of antigen processing and presentation of peptide antigen [GO:0002584]; RO_0002213 by positive regulation of antigen processing and presentation of peptide antigen [GO:0002585] Also known as: antigen presentation, peptide antigen, peptide antigen processing and presentation Relationships: is a type of antigen processing and presentation [GO:0019882] References: PMID:15771591 Sources: GOC:add, ISBN:0781735149 Subtypes: antigen processing and presentation of peptide antigen via MHC class Ib [GO:0002428], GO:0002474, antigen processing and presentation of exogenous peptide antigen [GO:0002478], GO:0002483, antigen processing and presentation of peptide antigen via MHC class II [GO:0002495]